nuclear envelope lumen [GO:0005641] (cellular component) Relationships: is a type of organelle envelope lumen [GO:0031970]; is part of nuclear envelope [GO:0005635] Definition: The region between the two lipid bilayers of the nuclear envelope; 20-40 nm wide. Also known as: nuclear intermembrane space, perinuclear space, nuclear membrane lumen Note: Note that this term should not be confused with the cellular component term 'perinuclear region ; GO:0048471'. Sources: GOC:ai